{
  "gene_name": "Phosphorylated adapter RNA export protein",
  "gene_symbol": "PHAX",
  "gene": "UniProtKB:Q9H814",
  "term_label": "snRNA export from nucleus",
  "term_id": "GO:0006408"
}